response to herbicide [GO:0009635] (biological process) Also known as: herbicide susceptibility/resistance Relationships: is a type of GO:0006950; is_a GO:0009636 Definition: Any process that results in a change in state or activity of a cell or an organism (in terms of movement, secretion, enzyme production, gene expression, etc.) as a result of a herbicide stimulus. Herbicides are chemicals used to kill or control the growth of plants. Sources: GOC:curators